{
  "gene": "UniProtKB:A8MTJ6",
  "term_id": "UNKNOWN:0003",
  "term_label": "Unknown cellular component",
  "gene_name": "Forkhead box protein I3",
  "gene_symbol": "FOXI3"
}